angelicin synthase activity [GO:0102995] (molecular function) Definition: Catalysis of the reaction: columbianetin + NADPH + O2 + H+ = angelicin + acetone + NADP + 2 H2O. Relationships: is a type of oxidoreductase activity, acting on paired donors, with incorporation or reduction of molecular oxygen, NAD(P)H as one donor, and incorporation of one atom of oxygen [GO:0016709] Sources: EC:1.14.14.148, GOC:pz